{
  "gene_symbol": "NME5",
  "term_id": "GO:1902176",
  "gene": "UniProtKB:P56597",
  "term_label": "negative regulation of oxidative stress-induced intrinsic apoptotic signaling pathway",
  "gene_name": "Nucleoside diphosphate kinase homolog 5"
}